regulation of macrophage inflammatory protein 1 alpha production [GO:0071640] (biological process) Subtypes: negative regulation of macrophage inflammatory protein 1 alpha production [GO:0071641], positive regulation of macrophage inflammatory protein 1 alpha production [GO:0071642] Also known as: regulation of macrophage inflammatory protein production, regulation of CCL3 production, regulation of MIP-1a production, regulation of chemokine (C-C motif) ligand 3 production Sources: GOC:mah Definition: Any process that modulates the frequency, rate, or extent of production of macrophage inflammatory protein 1 alpha. Relationships: is_a regulation of chemokine production [GO:0032642]; regulates macrophage inflammatory protein-1 alpha production [GO:0071608]